hydrolase activity, acting on ester bonds [GO:0016788] (molecular function) Also known as: esterase activity Sources: GOC:jl Relationships: is a type of hydrolase activity [GO:0016787] Definition: Catalysis of the hydrolysis of any ester bond. Subtypes: single-stranded DNA endodeoxyribonuclease activity [GO:0000014], ribonuclease MRP activity [GO:0000171], exonuclease activity [GO:0004527], GO:0008484, GO:0008849, excinuclease ABC activity [GO:0009381], restriction endodeoxyribonuclease activity [GO:0015666], lipase activity [GO:0016298], thiolester hydrolase activity [GO:0016790], DNA endonuclease activity, producing 5'-phosphomonoesters [GO:0016888], DNA endonuclease activity, producing 3'-phosphomonoesters [GO:0016889], GO:0016891, RNA endonuclease activity producing 3'-phosphomonoesters, hydrolytic mechanism [GO:0016892], double-stranded RNA-specific ribonuclease activity [GO:0032296], GO:0033892, phosphoric ester hydrolase activity [GO:0042578], retroviral 3' processing activity [GO:0044824], GO:0048256, GO:0052689, versiconal hemiacetal acetate esterase activity [GO:0140397], N-acetyltaurine hydrolase activity [GO:0141215], GO:1990238